{
  "term_id": "GO:0042613",
  "gene": "UniProtKB:Q30154",
  "gene_symbol": "HLA-DRB5",
  "gene_name": "HLA class II histocompatibility antigen, DR beta 5 chain",
  "term_label": "MHC class II protein complex"
}